{
  "term_id": "UNKNOWN:0002",
  "gene": "UniProtKB:Q0VFX4",
  "gene_symbol": "Q0VFX4",
  "term_label": "Unknown biological process",
  "gene_name": "Putative uncharacterized protein LOC100128554"
}